{
  "term_id": "GO:0003723",
  "term_label": "RNA binding",
  "gene": "UniProtKB:Q9HCE1",
  "gene_name": "Helicase MOV-10",
  "gene_symbol": "MOV10"
}